cellular response to folic acid [GO:0071231] (BP) Relationships: is a type of response to folic acid [GO:0051593]; is a type of GO:0071295; is a type of cellular response to nitrogen compound [GO:1901699]; is a type of cellular response to oxygen-containing compound [GO:1901701] Also known as: response to folate, response to vitamin B9 Definition: Any process that results in a change in state or activity of a cell (in terms of movement, secretion, enzyme production, gene expression, etc.) as a result of a folic acid stimulus. Sources: GOC:mah